deacetoxycephalosporin-C hydroxylase activity [GO:0045442] (molecular function) Sources: EC:1.14.11.26, RHEA:16805 Also known as: beta-lactam hydroxylase activity, 3'-methylcephem hydroxylase activity, DACS, DAOC hydroxylase activity, deacetoxycephalosporin C hydroxylase activity, deacetoxycephalosporin-C,2-oxoglutarate:oxygen oxidoreductase (3-hydroxylating) activity, deacetylcephalosporin C synthase activity Definition: Catalysis of the reaction: 2-oxoglutarate + deacetoxycephalosporin C + O2 = CO2 + deacetylcephalosporin C + succinate. Relationships: is a type of GO:0016706